{
  "gene_name": "DNA (cytosine-5)-methyltransferase 3B",
  "term_label": "nucleus",
  "gene": "UniProtKB:Q9UBC3",
  "gene_symbol": "DNMT3B",
  "term_id": "GO:0005634"
}